{
  "gene_name": "Double-strand-break repair protein rad21-like protein 1",
  "gene_symbol": "RAD21L1",
  "term_id": "GO:0030893",
  "term_label": "meiotic cohesin complex",
  "gene": "UniProtKB:Q9H4I0"
}